red or far-red light photoreceptor activity [GO:0009883] (molecular function) Relationships: is a type of photoreceptor activity [GO:0009881]; is part of red, far-red light phototransduction [GO:0009585] Also known as: red/far-red light photoreceptor activity Subtypes: GO:0031516, red light photoreceptor activity [GO:0031517] Definition: The function of absorbing and responding to electromagnetic radiation with a wavelength of approximately 660-730nm. The response may involve a change in conformation. Sources: GOC:lr